{
  "gene_symbol": "ZBTB4",
  "term_label": "regulation of DNA-templated transcription",
  "gene_name": "Zinc finger and BTB domain-containing protein 4",
  "gene": "UniProtKB:Q9P1Z0",
  "term_id": "GO:0006355"
}